{
  "term_label": "Unknown molecular function",
  "term_id": "UNKNOWN:0001",
  "gene_symbol": "ANKRD49",
  "gene_name": "Ankyrin repeat domain-containing protein 49",
  "gene": "UniProtKB:Q8WVL7"
}